{
  "gene_name": "Leucine-rich repeat and immunoglobulin-like domain-containing nogo receptor-interacting protein 2",
  "term_label": "plasma membrane",
  "gene_symbol": "LINGO2",
  "term_id": "GO:0005886",
  "gene": "UniProtKB:Q7L985"
}